positive regulation of ubiquitin-dependent endocytosis [GO:2000397] (biological process) Relationships: is a type of positive regulation of endocytosis [GO:0045807]; is a type of positive regulation of protein transport [GO:0051222]; is a type of regulation of ubiquitin-dependent endocytosis [GO:2000395]; RO_0002213 ubiquitin-dependent endocytosis [GO:0070086] Also known as: positive regulation of ubiquitin-mediated endocytosis Definition: Any process that activates or increases the frequency, rate or extent of ubiquitin-dependent endocytosis. Sources: GOC:mah